{
  "gene_symbol": "CCL28",
  "term_label": "CXCR chemokine receptor binding",
  "gene_name": "C-C motif chemokine 28",
  "gene": "UniProtKB:Q9NRJ3",
  "term_id": "GO:0045236"
}